{
  "gene_symbol": "TRBV5-8",
  "term_label": "cell surface receptor signaling pathway",
  "term_id": "GO:0007166",
  "gene_name": "T cell receptor beta variable 5-8",
  "gene": "UniProtKB:A0A5A2"
}